{
  "gene": "UniProtKB:O15455",
  "term_label": "signaling receptor activity",
  "gene_symbol": "TLR3",
  "gene_name": "Toll-like receptor 3",
  "term_id": "GO:0038023"
}